{
  "gene_name": "Transcriptional regulator ATRX",
  "term_id": "GO:0031490",
  "gene": "UniProtKB:P46100",
  "term_label": "chromatin DNA binding",
  "gene_symbol": "ATRX"
}